{
  "gene_name": "P antigen family member 3",
  "term_id": "UNKNOWN:0002",
  "gene_symbol": "PAGE3",
  "gene": "UniProtKB:Q5JUK9",
  "term_label": "Unknown biological process"
}